positive regulation of antigen receptor-mediated signaling pathway [GO:0050857] (biological process) Relationships: is a type of positive regulation of signal transduction [GO:0009967]; is a type of positive regulation of immune response [GO:0050778]; is a type of regulation of antigen receptor-mediated signaling pathway [GO:0050854]; positively regulates antigen receptor-mediated signaling pathway [GO:0050851] Also known as: positive regulation of antigen receptor mediated signalling pathway, up regulation of antigen receptor-mediated signaling pathway, up-regulation of antigen receptor-mediated signaling pathway, upregulation of antigen receptor-mediated signaling pathway, activation of antigen receptor-mediated signaling pathway, stimulation of antigen receptor-mediated signaling pathway Sources: GOC:ai Subtypes: positive regulation of B cell receptor signaling pathway [GO:0050861], GO:0050862 Definition: Any process that activates or increases the frequency, rate or extent of signaling pathways initiated by the cross-linking of an antigen receptor on a B- or T cell.